{
  "gene": "UniProtKB:P0CJ79",
  "gene_name": "Zinc finger protein 888",
  "gene_symbol": "ZNF888",
  "term_id": "GO:0000978",
  "term_label": "RNA polymerase II cis-regulatory region sequence-specific DNA binding"
}